lung epithelial cell differentiation [GO:0060487] (biological process) Definition: The process in which a relatively unspecialized cell acquires specialized features of an epithelial cell that contributes to the epithelium of the lung. Sources: GOC:dph Also known as: pulmonary epithelial cell differentiation Relationships: is a type of epithelial cell differentiation [GO:0030855]; is a type of lung cell differentiation [GO:0060479]; is part of GO:0060428 Subtypes: club cell differentiation [GO:0060486], type I pneumocyte differentiation [GO:0060509], lung secretory cell differentiation [GO:0061140], lung ciliated cell differentiation [GO:0061141]